alcohol metabolic process [GO:0006066] (biological process) Sources: ISBN:0198506732 Definition: The chemical reactions and pathways involving alcohols, any of a class of compounds containing one or more hydroxyl groups attached to a saturated carbon atom. Subtypes: polyprenol metabolic process [GO:0016093], 3-hydroxybenzyl alcohol metabolic process [GO:0018921], polyol metabolic process [GO:0019751], primary alcohol metabolic process [GO:0034308], alcohol catabolic process [GO:0046164], alcohol biosynthetic process [GO:0046165], octopamine metabolic process [GO:0046333], tertiary alcohol metabolic process [GO:1902644], secondary alcohol metabolic process [GO:1902652], fatty alcohol metabolic process [GO:1903173] Also known as: alcohol metabolism Relationships: is a type of GO:0044281